4-hydroxyphenylpyruvate dioxygenase activity [GO:0003868] (molecular function) Also known as: 4-hydroxyphenylpyruvate hydroxylase activity, 4-hydroxyphenylpyruvate:oxygen oxidoreductase (hydroxylating, decarboxylating), 4-hydroxyphenylpyruvic acid dioxygenase activity, p-hydroxyphenylpyruvate dioxygenase activity, p-hydroxyphenylpyruvate hydroxylase activity, p-hydroxyphenylpyruvate oxidase activity, p-hydroxyphenylpyruvic acid hydroxylase activity, p-hydroxyphenylpyruvic hydroxylase activity, p-hydroxyphenylpyruvic oxidase activity Sources: EC:1.13.11.27 Relationships: is a type of oxidoreductase activity, acting on single donors with incorporation of molecular oxygen, incorporation of two atoms of oxygen [GO:0016702] Definition: Catalysis of the reaction: 4-hydroxyphenylpyruvate + O2 = homogentisate + CO2.